{
  "gene_symbol": "GBX1",
  "gene_name": "Homeobox protein GBX-1",
  "term_label": "nucleus",
  "term_id": "GO:0005634",
  "gene": "UniProtKB:Q14549"
}